{
  "term_id": "GO:0005737",
  "gene": "UniProtKB:Q09666",
  "gene_name": "Neuroblast differentiation-associated protein AHNAK",
  "term_label": "cytoplasm",
  "gene_symbol": "AHNAK"
}